{
  "gene": "UniProtKB:C9JPN9",
  "gene_name": "Ubiquitin carboxyl-terminal hydrolase 17-like protein 12",
  "term_label": "nucleus",
  "gene_symbol": "USP17L12",
  "term_id": "GO:0005634"
}